{
  "term_id": "GO:0005520",
  "gene_name": "Insulin-like growth factor-binding protein complex acid labile subunit",
  "gene_symbol": "IGFALS",
  "gene": "UniProtKB:P35858",
  "term_label": "insulin-like growth factor binding"
}